acetylenecarboxylate hydratase activity [GO:0050079] (molecular function) Sources: RHEA:17957 Also known as: acetylenemonocarboxylate hydratase activity, alkynoate hydratase activity, acetylenecarboxylate hydratase activity, producing malonate-semialdehyde, 3-oxopropanoate hydro-lyase (propynoate-forming), 3-oxopropanoate hydro-lyase activity, acetylenemonocarboxylate hydrase activity, acetylmonocarboxylic acid hydrase activity, malonate-semialdehyde dehydratase activity Relationships: is a type of hydro-lyase activity [GO:0016836] Definition: Catalysis of the reaction: 3-oxopropanoate = propynoate + H2O.